{
  "gene_name": "Protein LLP homolog",
  "term_label": "dendrite extension",
  "gene": "UniProtKB:Q9BRT6",
  "term_id": "GO:0097484",
  "gene_symbol": "LLPH"
}